juxtaglomerulus cell fate commitment [GO:0072150] (biological process) Subtypes: mesonephric juxtaglomerulus cell fate commitment [GO:0061230], metanephric juxtaglomerulus cell fate commitment [GO:0072253] Relationships: is a type of cell fate commitment [GO:0045165]; is part of juxtaglomerulus cell differentiation [GO:0072052] Definition: The process in which the developmental fate of a cell becomes restricted such that it will develop into a juxtaglomerulus cell. Sources: GOC:mtg_kidney_jan10